reactive-black-5:hydrogen-peroxide oxidoreductase activity [GO:0052750] (molecular function) Definition: Catalysis of the reaction: reactive black 5 + hydrogen peroxide = oxidized reactive black 5 + 2 H2O. Sources: KEGG_REACTION:R07612, MetaCyc:RXN-8666 Also known as: versatile peroxidase activity Relationships: is a type of peroxidase activity [GO:0004601]